{
  "gene": "UniProtKB:Q99471",
  "gene_name": "Prefoldin subunit 5",
  "term_id": "GO:0005737",
  "term_label": "cytoplasm",
  "gene_symbol": "PFDN5"
}